negative regulation of cell septum assembly [GO:1901892] (biological process) Subtypes: negative regulation of division septum assembly [GO:0010974] Also known as: down regulation of cell septum assembly, down-regulation of cell septum assembly, downregulation of cell septum assembly, inhibition of cell septum assembly Definition: Any process that stops, prevents or reduces the frequency, rate or extent of cell septum assembly. Relationships: is a type of negative regulation of cytokinesis [GO:0032466]; is a type of GO:0051129; is a type of regulation of cell septum assembly [GO:1901891]; negatively regulates cell septum assembly [GO:0090529] Sources: GOC:TermGenie